regulation of signaling receptor activity [GO:0010469] (biological process) Definition: Any process that modulates the frequency, rate or extent of a signaling receptor activity. Receptor activity is when a molecule combines with an extracellular or intracellular messenger to initiate a change in cell activity. Sources: GOC:dph, GOC:tb Subtypes: regulation of nerve growth factor receptor activity [GO:0051394], regulation of cytokine activity [GO:0060300], GO:0099601, regulation of GABA-A receptor activity [GO:0106040], negative regulation of signaling receptor activity [GO:2000272], positive regulation of androgen receptor activity [GO:2000825] Also known as: regulation of receptor activity, regulation of signalling receptor activity Relationships: is a type of GO:0009966; is a type of regulation of molecular function [GO:0065009]; regulates signaling receptor activity [GO:0038023]